{
  "term_id": "GO:0017056",
  "term_label": "structural constituent of nuclear pore",
  "gene_name": "Nucleoporin p58_p45",
  "gene_symbol": "NUP58",
  "gene": "UniProtKB:Q9BVL2"
}